{
  "gene_name": "Coiled-coil domain-containing protein 9",
  "term_label": "Unknown biological process",
  "gene": "UniProtKB:Q9Y3X0",
  "gene_symbol": "CCDC9",
  "term_id": "UNKNOWN:0002"
}